{
  "term_id": "UNKNOWN:0001",
  "term_label": "Unknown molecular function",
  "gene": "UniProtKB:Q9UBQ6",
  "gene_name": "Exostosin-like 2",
  "gene_symbol": "EXTL2"
}